{
  "term_label": "plasma membrane",
  "term_id": "GO:0005886",
  "gene": "UniProtKB:P07359",
  "gene_name": "Platelet glycoprotein Ib alpha chain",
  "gene_symbol": "GP1BA"
}